{
  "gene_symbol": "TEX14",
  "term_id": "GO:0008608",
  "term_label": "attachment of spindle microtubules to kinetochore",
  "gene_name": "Inactive serine_threonine-protein kinase TEX14",
  "gene": "UniProtKB:Q8IWB6"
}